sorbose reductase activity [GO:0032115] (molecular function) Sources: EC:1.1.1.289, RHEA:14609 Relationships: is a type of GO:0016616 Definition: Catalysis of the reaction: D-glucitol + NADP+ = L-sorbose + H+ + NADPH. The reaction may occur, to a minor extent, in the reverse direction. Also known as: D-glucitol:NADP+ oxidoreductase activity, Sou1p